negative regulation of uracil import across plasma membrane [GO:1905530] (biological process) Relationships: is a type of negative regulation of transmembrane transport [GO:0034763]; is a type of regulation of uracil import across plasma membrane [GO:1905529]; negatively regulates uracil import across plasma membrane [GO:0098721] Definition: Any process that stops, prevents or reduces the frequency, rate or extent of uracil import across plasma membrane. References: PMID:26536126 Sources: GOC:TermGenie, GO_REF:0000058